{
  "gene_name": "Solute carrier family 12 member 8",
  "gene_symbol": "SLC12A8",
  "gene": "UniProtKB:A0AV02",
  "term_id": "UNKNOWN:0003",
  "term_label": "Unknown cellular component"
}